sucrase-isomaltase complex [GO:0070014] (cellular component) Definition: A protein complex that possesses oligo-1,6-glucosidase activity; the complex is a heterodimer located in the cell membrane, and is formed by proteolytic cleavage of a single precursor polypeptide. The two subunits have different substrate specificities. Relationships: is_a GO:0098797; is a type of glucosidase complex [GO:1902687] Also known as: oligo-1,6-glucosidase complex References: PMID:3366777